{
  "gene": "UniProtKB:Q9Y6M4",
  "gene_symbol": "CSNK1G3",
  "gene_name": "Casein kinase I isoform gamma-3",
  "term_label": "positive regulation of canonical Wnt signaling pathway",
  "term_id": "GO:0090263"
}